inner ear sensory epithelium regeneration [GO:0070659] (biological process) Relationships: is a type of GO:0070655 Definition: The regrowth of lost or destroyed inner ear sensory epithelia. References: PMID:19381250 Sources: GOC:dsf